{
  "term_id": "GO:0034702",
  "gene_symbol": "LRRC8A",
  "term_label": "monoatomic ion channel complex",
  "gene": "UniProtKB:Q8IWT6",
  "gene_name": "Volume-regulated anion channel subunit LRRC8A"
}